{
  "term_label": "midbody",
  "gene_symbol": "MPLKIP",
  "gene_name": "M-phase-specific PLK1-interacting protein",
  "term_id": "GO:0030496",
  "gene": "UniProtKB:Q8TAP9"
}